{
  "term_label": "regulation of transcription by RNA polymerase II",
  "gene_symbol": "MAMLD1",
  "term_id": "GO:0006357",
  "gene": "UniProtKB:Q13495",
  "gene_name": "Mastermind-like domain-containing protein 1"
}